{
  "term_label": "regulation of transcription by RNA polymerase II",
  "term_id": "GO:0006357",
  "gene_name": "Zinc finger protein 517",
  "gene": "UniProtKB:Q6ZMY9",
  "gene_symbol": "ZNF517"
}